{
  "gene_name": "NAD-dependent protein deacetylase sirtuin-7",
  "term_label": "protein-succinyllysine desuccinylase activity",
  "gene_symbol": "SIRT7",
  "gene": "UniProtKB:Q9NRC8",
  "term_id": "GO:0036055"
}